{
  "term_id": "UNKNOWN:0001",
  "gene_symbol": "ENTPD5",
  "term_label": "Unknown molecular function",
  "gene_name": "Nucleoside diphosphate phosphatase ENTPD5",
  "gene": "UniProtKB:O75356"
}